{
  "term_id": "GO:0001788",
  "gene_symbol": "FCGR1A",
  "gene": "UniProtKB:P12314",
  "term_label": "antibody-dependent cellular cytotoxicity",
  "gene_name": "High affinity immunoglobulin gamma Fc receptor I"
}